proteinogenic amino acid biosynthetic process [GO:0170038] (BP) Subtypes: GO:0000105, L-tryptophan biosynthetic process [GO:0000162], glycine biosynthetic process [GO:0006545], L-serine biosynthetic process [GO:0006564], L-tyrosine biosynthetic process [GO:0006571], aspartate family amino acid biosynthetic process [GO:0009067], pyruvate family amino acid biosynthetic process [GO:0009079], GO:0009084, L-phenylalanine biosynthetic process [GO:0009094], pyrrolysine biosynthetic process [GO:0071524] Relationships: is a type of carboxylic acid biosynthetic process [GO:0046394]; is a type of GO:0170039 Sources: GOC:ew Definition: The chemical reactions and pathways resulting in the formation of any amino acid that is incorporated into protein naturally by ribosomal translation of mRNA, and that has a specific codon for translation from mRNA to protein. Also known as: proteinogenic amino acid anabolism, proteinogenic amino acid biosynthesis, proteinogenic amino acid formation, proteinogenic amino acid synthesis